{
  "term_id": "GO:0005737",
  "gene": "UniProtKB:P27482",
  "gene_name": "Calmodulin-like protein 3",
  "term_label": "cytoplasm",
  "gene_symbol": "CALML3"
}